{
  "term_label": "protein serine/threonine phosphatase inhibitor activity",
  "gene_symbol": "PPP1R14B",
  "gene": "UniProtKB:Q96C90",
  "gene_name": "Protein phosphatase 1 regulatory subunit 14B",
  "term_id": "GO:0004865"
}